tensidol A catabolic process [GO:1900604] (biological process) Relationships: is a type of ketone catabolic process [GO:0042182]; is a type of amide metabolic process [GO:0043603]; is a type of secondary metabolite catabolic process [GO:0090487] Definition: The chemical reactions and pathways resulting in the breakdown of tensidol A. Also known as: tensidol A breakdown, tensidol A catabolism, tensidol A degradation Sources: GOC:TermGenie, GOC:di